regulation of urothelial cell proliferation [GO:0050675] (biological process) Sources: GOC:ai Subtypes: negative regulation of urothelial cell proliferation [GO:0050676], positive regulation of urothelial cell proliferation [GO:0050677] Definition: Any process that modulates the frequency, rate or extent of urothelial cell proliferation. Relationships: is a type of regulation of epithelial cell proliferation [GO:0050678]; regulates urothelial cell proliferation [GO:0050674]